{
  "gene_symbol": "NOS1",
  "term_id": "GO:0005634",
  "gene_name": "Nitric oxide synthase 1",
  "term_label": "nucleus",
  "gene": "UniProtKB:P29475"
}